{
  "gene": "UniProtKB:Q99856",
  "term_id": "GO:0006357",
  "gene_name": "AT-rich interactive domain-containing protein 3A",
  "term_label": "regulation of transcription by RNA polymerase II",
  "gene_symbol": "ARID3A"
}